{
  "term_id": "GO:0097225",
  "gene": "UniProtKB:Q7Z5L4",
  "gene_symbol": "SPATA19",
  "term_label": "sperm midpiece",
  "gene_name": "Spermatogenesis-associated protein 19, mitochondrial"
}